{
  "term_id": "GO:0048699",
  "term_label": "generation of neurons",
  "gene": "UniProtKB:Q8N3R9",
  "gene_name": "Protein PALS1",
  "gene_symbol": "PALS1"
}